{
  "term_label": "structural constituent of chromatin",
  "gene_symbol": "H2AC14",
  "gene": "UniProtKB:Q99878",
  "gene_name": "Histone H2A type 1-J",
  "term_id": "GO:0030527"
}